O-methyltransferase activity [GO:0008171] (molecular function) Subtypes: methyltransferase cap1 activity [GO:0004483], carboxyl-O-methyltransferase activity [GO:0010340], catechol O-methyltransferase activity [GO:0016206], GO:0017096, farnesoic acid O-methyltransferase activity [GO:0019010], myricetin 3'-O-methyltransferase activity [GO:0033799], isoflavone 7-O-methyltransferase activity [GO:0033800], vitexin 2''-O-rhamnoside 7-O-methyltransferase activity [GO:0033801], isoliquiritigenin 2'-O-methyltransferase activity [GO:0033802], GO:0033803, caffeoyl-CoA O-methyltransferase activity [GO:0042409], magnesium protoporphyrin IX methyltransferase activity [GO:0046406], demethylsterigmatocystin 6-O-methyltransferase activity [GO:0047145], sterigmatocystin 7-O-methyltransferase activity [GO:0047146], caffeate O-methyltransferase activity [GO:0047763], tocopherol C-methyltransferase activity [GO:0050342], (iso)eugenol O-methyltransferase activity [GO:0050630], GO:0052624, 3-demethylubiquinol 3-O-methyltransferase activity [GO:0061542], RNA 2'-O-methyltransferase activity [GO:0062105], GO:0070448, trihydroxyferuloyl spermidine O-methyltransferase activity [GO:0080012], trihydroxyferuloyl spermidine:S-adenosyl-L-methionine O-methyltransferase activity [GO:0080077], tricaffeoyl spermidine:S-adenosyl-L-methionine O-methyltransferase activity [GO:0080078], GO:0080150, flavone 3'-O-methyltransferase activity [GO:0102822], 3-demethylubiquinone 3-O-methyltransferase activity [GO:0120537], methyltransferase cap2 activity [GO:0120550], 4-vinylphenol methyltransferase activity [GO:0160304], GO:1990276, GO:1990888 Definition: Catalysis of the transfer of a methyl group to the oxygen atom of an acceptor molecule. Sources: GOC:ai Relationships: is a type of methyltransferase activity [GO:0008168]